{
  "gene": "UniProtKB:Q9Y6R4",
  "term_label": "Unknown cellular component",
  "term_id": "UNKNOWN:0003",
  "gene_name": "Mitogen-activated protein kinase kinase kinase 4",
  "gene_symbol": "MAP3K4"
}